{
  "gene_symbol": "ORC6",
  "gene": "UniProtKB:Q9Y5N6",
  "term_label": "nuclear origin of replication recognition complex",
  "gene_name": "Origin recognition complex subunit 6",
  "term_id": "GO:0005664"
}